{
  "term_label": "Unknown biological process",
  "gene_name": "Mitochondrial S-adenosylmethionine carrier protein",
  "term_id": "UNKNOWN:0002",
  "gene_symbol": "SLC25A26",
  "gene": "UniProtKB:Q70HW3"
}